{
  "gene_symbol": "NUDT4",
  "gene_name": "Diphosphoinositol polyphosphate phosphohydrolase 2",
  "term_id": "GO:0005737",
  "gene": "UniProtKB:Q9NZJ9",
  "term_label": "cytoplasm"
}